{
  "term_id": "GO:0005634",
  "gene": "UniProtKB:P05413",
  "gene_symbol": "FABP3",
  "term_label": "nucleus",
  "gene_name": "Fatty acid-binding protein, heart"
}